{
  "term_id": "GO:0030672",
  "gene": "UniProtKB:O95670",
  "term_label": "synaptic vesicle membrane",
  "gene_name": "V-type proton ATPase subunit G 2",
  "gene_symbol": "ATP6V1G2"
}